{
  "term_label": "Unknown cellular component",
  "gene_name": "P antigen family member 2",
  "term_id": "UNKNOWN:0003",
  "gene_symbol": "PAGE2",
  "gene": "UniProtKB:Q7Z2X7"
}